mannosylphosphate transferase activity [GO:0000031] (molecular function) Relationships: is a type of hexosyltransferase activity [GO:0016758] Definition: Catalysis of the reaction: GDP-alpha-D-mannose + n {[alpha-D-Man-(1->2)-alpha-D-Man-(1->2)]-alpha-D-Man-(1->6)}60-(Man9GlcNAc2-[protein] = phosphorylated {[alpha-D-Man-(1->2)-alpha-D-Man-(1->2)]-alpha-D-Man-(1->6)}60-(Man9GlcNAc2-[protein] + n GMP + n H+ or GDP-alpha-D-mannose + alpha-D-Man-(1->3)-alpha-D-Man-(1->3)-alpha-D-Man-(1->2)-alpha-D-Man-(1->2)-alpha-D-Man-3-O-(Ser/Thr)-[protein] = alpha-D-Man-(1->3)-alpha-D-Man-(1->3)-[alpha-D-Man-6P-]-alpha-D-Man-(1->2)-alpha-D-Man-(1->2)-alpha-D-Man-3-O-(Ser/Thr)-[protein] + GMP + H+. Sources: MetaCyc:RXN-22693, MetaCyc:RXN-22694